{
  "gene_name": "Nuclear receptor ROR-alpha",
  "term_label": "regulation of transcription by RNA polymerase II",
  "gene": "UniProtKB:P35398",
  "gene_symbol": "RORA",
  "term_id": "GO:0006357"
}